{
  "term_id": "GO:0005886",
  "gene": "UniProtKB:Q9H3S3",
  "gene_symbol": "TMPRSS5",
  "gene_name": "Transmembrane protease serine 5",
  "term_label": "plasma membrane"
}